{
  "term_label": "Unknown molecular function",
  "gene": "UniProtKB:Q9Y2G4",
  "gene_name": "Ankyrin repeat domain-containing protein 6",
  "term_id": "UNKNOWN:0001",
  "gene_symbol": "ANKRD6"
}